{
  "gene_name": "Double-stranded RNA-binding protein Staufen homolog 1",
  "gene_symbol": "STAU1",
  "term_label": "double-stranded RNA binding",
  "term_id": "GO:0003725",
  "gene": "UniProtKB:O95793"
}